gamma-tubulin small complex [GO:0008275] (cellular component) References: PMID:11297925, PMID:12134075 Relationships: is a type of gamma-tubulin complex [GO:0000930] Also known as: gammaTuSC, Tub4 complex, gamma-tubulin small complex, centrosomal, gamma-tubulin small complex, mitotic spindle pole body, gamma-tubulin small complex, spindle pole body Definition: A complex usually comprising two gamma-tubulin molecules and two conserved non-tubulin proteins. Some gamma-tubulin small complexes are thought to be the repeating unit making up the core of the gamma-tubulin ring complex.